{
  "term_label": "regulation of transcription by RNA polymerase II",
  "term_id": "GO:0006357",
  "gene": "UniProtKB:Q0VGE8",
  "gene_symbol": "ZNF816",
  "gene_name": "Zinc finger protein 816"
}